{
  "gene_name": "E3 ubiquitin-protein ligase RNF146",
  "term_id": "GO:0006511",
  "gene_symbol": "RNF146",
  "gene": "UniProtKB:Q9NTX7",
  "term_label": "ubiquitin-dependent protein catabolic process"
}